{
  "gene": "UniProtKB:Q7Z7L9",
  "term_label": "DNA-binding transcription factor activity, RNA polymerase II-specific",
  "gene_symbol": "ZSCAN2",
  "gene_name": "Zinc finger and SCAN domain-containing protein 2",
  "term_id": "GO:0000981"
}